tachykinin receptor activity [GO:0004995] (molecular function) Definition: Combining with a tachykinin neuropeptide and transmitting the signal across the membrane by activating an associated G-protein. References: PMID:7639617 Sources: GOC:ai, GOC:bf, Wikipedia:Tachykinin Relationships: is a type of neuropeptide receptor activity [GO:0008188]; is part of GO:0007217 Subtypes: GO:0016496, substance K receptor activity [GO:0016497], neuromedin K receptor activity [GO:0016498]